{
  "term_label": "RNA binding",
  "gene_symbol": "RALY",
  "term_id": "GO:0003723",
  "gene": "UniProtKB:Q9UKM9",
  "gene_name": "RNA-binding protein Raly"
}